{
  "gene": "UniProtKB:Q86UY8",
  "gene_name": "5'-nucleotidase domain-containing protein 3",
  "term_label": "5'-nucleotidase activity",
  "gene_symbol": "NT5DC3",
  "term_id": "GO:0008253"
}